{
  "gene_name": "E3 ubiquitin-protein ligase TRIM23",
  "gene_symbol": "TRIM23",
  "term_label": "intracellular protein transport",
  "term_id": "GO:0006886",
  "gene": "UniProtKB:P36406"
}